{
  "gene": "UniProtKB:Q92834",
  "term_id": "GO:0061630",
  "term_label": "ubiquitin protein ligase activity",
  "gene_name": "X-linked retinitis pigmentosa GTPase regulator",
  "gene_symbol": "RPGR"
}